glycine cleavage complex [GO:0005960] (cellular component) Sources: GOC:mah Relationships: is a type of oxidoreductase complex [GO:1990204]; is a type of transferase complex [GO:1990234] Also known as: glycine cleavage system, glycine decarboxylase complex, glycine dehydrogenase (decarboxylating) complex, glycine synthase complex, glycine dehydrogenase complex (decarboxylating) Definition: A protein complex that catalyzes the reversible oxidation of glycine. In E. coli, it has four components: dihydrolipoamide dehydrogenase, glycine dehydrogenase (decarboxylating), lipoyl-GcvH-protein and aminomethyltransferase, also known as L, P, H, and T.